response to nitrite [GO:0080033] (biological process) References: PMID:17951451 Sources: GOC:dhl Relationships: is a type of GO:1901698; is a type of response to oxygen-containing compound [GO:1901700] Definition: Any process that results in a change in state or activity of a cell or an organism (in terms of movement, secretion, enzyme production, gene expression, etc.) as a result of a nitrite stimulus. Subtypes: cellular response to nitrite [GO:0071250]